UDP-glucosamine 4-epimerase activity [GO:0050376] (molecular function) Definition: Catalysis of the reaction: UDP-glucosamine = UDP-galactosamine. Also known as: UDP-glucosamine epimerase activity, UDPglucosamine 4-epimerase activity Sources: EC:5.1.3.16, MetaCyc:UDP-GLUCOSAMINE-EPIMERASE-RXN Relationships: is a type of racemase and epimerase activity, acting on carbohydrates and derivatives [GO:0016857]